{
  "gene": "UniProtKB:P0CI01",
  "term_id": "UNKNOWN:0003",
  "term_label": "Unknown cellular component",
  "gene_name": "Speedy protein E6",
  "gene_symbol": "SPDYE6"
}